long-chain fatty acid-CoA ligase activity [GO:0004467] (molecular function) Also known as: acyl-activating enzyme activity, long-chain acyl-CoA synthetase activity, long-chain-fatty-acid-CoA ligase activity, long-chain-fatty-acyl-CoA synthetase activity, pristanoyl-CoA synthetase, stearoyl-CoA synthetase, LCFA synthetase activity, acyl-CoA ligase activity, acyl-CoA synthetase activity, fatty acid thiokinase (long-chain) activity, lignoceroyl-CoA synthase activity, long chain fatty acyl-CoA synthetase activity, long-chain acyl CoA synthetase activity, long-chain acyl-coenzyme A synthetase activity, long-chain fatty acid activation, long-chain fatty acyl coenzyme A synthetase activity, thiokinase Definition: Catalysis of the reaction: a long-chain fatty acid + ATP + CoA = a long-chain fatty acyl-CoA + AMP + diphosphate. A long-chain fatty acid has an aliphatic tail containing 13 to 22 carbons. Note: While there is not universal consensus on the lengths of short-, medium-, long- and very-long-chain fatty acids, the GO uses the definitions in ChEBI (see CHEBI:26666, CHEBI:59554, CHEBI:15904 and CHEBI:27283). Note that this term has a MetaCyc pathway reference as the pathway only has a single step. Relationships: is a type of fatty acid-CoA ligase activity [GO:0120515]; is part of long-chain fatty acid metabolic process [GO:0001676] Subtypes: arachidonate-CoA ligase activity [GO:0047676], myristoyl-CoA ligase activity [GO:0090432], palmitoyl-CoA ligase activity [GO:0090433], oleoyl-CoA ligase activity [GO:0090434] Sources: RHEA:15421